structural constituent of cell wall [GO:0005199] (molecular function) Subtypes: GO:1990915 Sources: GOC:mah Relationships: is a type of structural molecule activity [GO:0005198]; occurs in cell wall [GO:0005618] Definition: The action of a molecule that contributes to the structural integrity of a cell wall.